induction of conjugation upon carbon starvation [GO:0031141] (biological process) Sources: GOC:mah Relationships: is a type of induction of conjugation upon nutrient starvation [GO:0031140] Definition: The process in which a cell initiates conjugation with cellular fusion upon carbon starvation.